cellular response to cyanide [GO:1903928] (biological process) References: PMID:21854848 Sources: GOC:TermGenie, GO_REF:0000071 Definition: Any process that results in a change in state or activity of a cell (in terms of movement, secretion, enzyme production, gene expression, etc.) as a result of a cyanide stimulus. Relationships: is a type of cellular response to chemical stimulus [GO:0070887]; is a type of GO:1903927